{
  "gene": "UniProtKB:A0A1W2PPD8",
  "term_label": "chromatin",
  "gene_name": "Probable lysine-specific demethylase 4F",
  "term_id": "GO:0000785",
  "gene_symbol": "KDM4F"
}